{
  "gene": "UniProtKB:P08648",
  "gene_symbol": "ITGA5",
  "term_label": "cell surface",
  "gene_name": "Integrin alpha-5",
  "term_id": "GO:0009986"
}